{
  "gene_name": "Leucine-rich repeat serine_threonine-protein kinase 2",
  "gene_symbol": "LRRK2",
  "term_label": "regulation of dopamine receptor signaling pathway",
  "term_id": "GO:0060159",
  "gene": "UniProtKB:Q5S007"
}